{
  "gene_name": "IQ domain-containing protein N",
  "gene": "UniProtKB:Q9H0B3",
  "term_label": "Unknown molecular function",
  "term_id": "UNKNOWN:0001",
  "gene_symbol": "IQCN"
}